intracellular cyclic nucleotide activated cation channel complex [GO:0017071] (cellular component) Sources: GOC:mah Relationships: is a type of cation channel complex [GO:0034703] Definition: A protein complex that forms a transmembrane channel through which cations ions may pass in response to an intracellular cyclic nucleotide binding to the channel complex or one of its constituent parts.